{
  "gene_name": "Large ribosomal subunit protein uL18",
  "gene": "UniProtKB:P46777",
  "gene_symbol": "RPL5",
  "term_id": "GO:0008097",
  "term_label": "5S rRNA binding"
}